{
  "term_label": "odorant binding",
  "term_id": "GO:0005549",
  "gene_symbol": "OR5D16",
  "gene_name": "Olfactory receptor 5D16",
  "gene": "UniProtKB:Q8NGK9"
}